{
  "gene_name": "5-hydroxytryptamine receptor 1F",
  "term_id": "GO:0007198",
  "gene": "UniProtKB:P30939",
  "term_label": "adenylate cyclase-inhibiting serotonin receptor signaling pathway",
  "gene_symbol": "HTR1F"
}